dendrite cytoplasm [GO:0032839] (cellular component) Relationships: is_a GO:0120111; is part of dendrite [GO:0030425] Also known as: dendritic cytoplasm Subtypes: dendritic spine cytoplasm [GO:0061846] Sources: GOC:mah Definition: All of the contents of a dendrite, excluding the surrounding plasma membrane.